{
  "gene": "UniProtKB:Q8NCS7",
  "term_id": "GO:0055085",
  "gene_name": "Choline transporter-like protein 5",
  "gene_symbol": "SLC44A5",
  "term_label": "transmembrane transport"
}